response to L-ascorbic acid [GO:0033591] (BP) Relationships: is_a GO:0033273; is a type of response to monosaccharide [GO:0034284] Also known as: response to ascorbic acid, response to L-ascorbate, response to vitamin C Subtypes: GO:0071298 Sources: GOC:sl Definition: Any process that results in a change in state or activity of a cell or an organism (in terms of movement, secretion, enzyme production, gene expression, etc.) as a result of an L-ascorbic acid (vitamin C) stimulus.